{
  "gene_symbol": "LAMTOR4",
  "term_label": "cellular response to amino acid stimulus",
  "term_id": "GO:0071230",
  "gene_name": "Ragulator complex protein LAMTOR4",
  "gene": "UniProtKB:Q0VGL1"
}